{
  "gene_name": "mRNA-capping enzyme",
  "gene_symbol": "RNGTT",
  "term_label": "Unknown cellular component",
  "term_id": "UNKNOWN:0003",
  "gene": "UniProtKB:O60942"
}